response to ether [GO:0045472] (BP) Definition: Any process that results in a change in state or activity of a cell or an organism (in terms of movement, secretion, enzyme production, gene expression, etc.) as a result of a ether stimulus. Sources: GOC:go_curators Relationships: is a type of response to oxygen-containing compound [GO:1901700] Subtypes: response to iloperidone [GO:0036287], cellular response to ether [GO:0071362], response to trichodermin [GO:1901324], response to rapamycin [GO:1901355], response to diphenyl ether [GO:1901497], response to fenofibrate [GO:1901557], response to tamsulosin [GO:1901905], response to differentiation-inducing factor 1 [GO:1903013], GO:1904316, GO:1904558, response to ionomycin [GO:1904636], response to curcumin [GO:1904643], response to differentiation-inducing factor 2 [GO:1905960]